{
  "term_label": "mitochondrial ATP transmembrane transport",
  "gene_name": "ADP_ATP translocase 2",
  "gene_symbol": "SLC25A5",
  "gene": "UniProtKB:P05141",
  "term_id": "GO:1990544"
}